3'-UTR-mediated mRNA destabilization [GO:0061158] (biological process) Sources: GOC:dph, GOC:jh Definition: An mRNA destabilization process in which one or more RNA-binding proteins associate with the 3'-untranslated region (UTR) of an mRNA. Relationships: is a type of GO:0061157